plasmacytoid dendritic cell cytokine production [GO:0002373] (BP) Regulation: regulated by regulation of plasmacytoid dendritic cell cytokine production [GO:0002736]; negatively regulated by negative regulation of plasmacytoid dendritic cell cytokine production [GO:0002737]; positively regulated by positive regulation of plasmacytoid dendritic cell cytokine production [GO:0002738] Relationships: is a type of dendritic cell cytokine production [GO:0002371] Note: Note that this term is in the subset of terms that should not be used for direct gene product annotation. Instead, select one of the 'regulation' children terms. Definition: Any process that contributes to cytokine production by a plasmacytoid dendritic cell. Sources: GOC:add, ISBN:0781735149